{
  "gene_symbol": "EPPK1",
  "gene": "UniProtKB:P58107",
  "term_id": "GO:0005198",
  "gene_name": "Epiplakin",
  "term_label": "structural molecule activity"
}